G protein-coupled acetylcholine receptor signaling pathway involved in positive regulation of acetylcholine secretion, neurotransmission [GO:1904065] (BP) Relationships: is a type of G protein-coupled acetylcholine receptor signaling pathway [GO:0007213]; BFO_0000050 GO:0014057 Definition: Any G protein-coupled acetylcholine receptor signaling pathway that is involved in positive regulation of acetylcholine secretion, neurotransmission. References: PMID:22588719 Sources: GOC:TermGenie, GOC:kmv, GO_REF:0000060 Also known as: G-protein coupled acetylcholine receptor signaling pathway involved in positive regulation of acetylcholine secretion, neurotransmission, G-protein coupled acetylcholine receptor signaling pathway involved in up regulation of acetylcholine secretion, G-protein coupled acetylcholine receptor signaling pathway involved in up-regulation of acetylcholine secretion, G-protein coupled acetylcholine receptor signaling pathway involved in upregulation of acetylcholine secretion, acetylcholine receptor signalling, muscarinic pathway involved in positive regulation of acetylcholine secretion, neurotransmission, acetylcholine receptor signalling, muscarinic pathway involved in up regulation of acetylcholine secretion, acetylcholine receptor signalling, muscarinic pathway involved in up-regulation of acetylcholine secretion, acetylcholine receptor signalling, muscarinic pathway involved in upregulation of acetylcholine secretion, muscarinic acetylcholine receptor signaling pathway involved in positive regulation of acetylcholine secretion, neurotransmission, muscarinic acetylcholine receptor signaling pathway involved in up regulation of acetylcholine secretion, muscarinic acetylcholine receptor signaling pathway involved in up-regulation of acetylcholine secretion, muscarinic acetylcholine receptor signaling pathway involved in upregulation of acetylcholine secretion, G-protein coupled acetylcholine receptor signaling pathway involved in activation of acetylcholine secretion, G-protein coupled acetylcholine receptor signaling pathway involved in stimulation of acetylcholine secretion, acetylcholine receptor signalling, muscarinic pathway involved in activation of acetylcholine secretion, acetylcholine receptor signalling, muscarinic pathway involved in stimulation of acetylcholine secretion, muscarinic acetylcholine receptor signaling pathway involved in activation of acetylcholine secretion, muscarinic acetylcholine receptor signaling pathway involved in stimulation of acetylcholine secretion